{
  "gene_symbol": "COPS8",
  "term_label": "Unknown biological process",
  "gene": "UniProtKB:Q99627",
  "gene_name": "COP9 signalosome complex subunit 8",
  "term_id": "UNKNOWN:0002"
}